{
  "gene_name": "Junctional adhesion molecule-like",
  "gene": "UniProtKB:Q86YT9",
  "gene_symbol": "JAML",
  "term_id": "GO:0007157",
  "term_label": "heterophilic cell-cell adhesion"
}